aspartate-semialdehyde dehydrogenase activity [GO:0004073] (molecular function) Sources: EC:1.2.1.11, RHEA:24284 Relationships: is a type of oxidoreductase activity, acting on the aldehyde or oxo group of donors, NAD or NADP as acceptor [GO:0016620] Also known as: ASA dehydrogenase activity, L-aspartate-4-semialdehyde:NADP+ oxidoreductase (phosphorylating), L-aspartate-beta-semialdehyde dehydrogenase activity, L-aspartate-beta-semialdehyde:NADP oxidoreductase (phosporylating), aspartate semialdehyde dehydrogenase activity, aspartic beta-semialdehyde dehydrogenase activity, aspartic semialdehyde dehydrogenase activity Definition: Catalysis of the reaction: L-aspartate 4-semialdehyde + NADP+ + phosphate = 4-phospho-L-aspartate + H+ + NADPH.